corneocyte development [GO:0003335] (biological process) Definition: The process whose specific outcome is the progression of the corneocyte over time, from its formation to the mature structure. A corneocyte is the last stage of development of a keratinocyte where the keratinocyte flattens, loses its nucleus and eventually delaminates from the epidermis. Sources: GOC:dph Relationships: is a type of cell development [GO:0048468]; is part of keratinocyte development [GO:0003334]